interleukin-1, type II, blocking receptor activity [GO:0004910] (molecular function) Definition: Combining with interleukin-1 to initiate a change in cell activity by inhibiting the activity of type I interleukin receptors. References: PMID:15062641, PMID:18613828 Also known as: IL-1 type II, blocking binding, IL-1 type II, blocking receptor, interleukin-1 blocking receptor activity, interleukin-1 type II receptor activity, interleukin-1, type II, blocking binding Relationships: is a type of interleukin-1 receptor activity [GO:0004908]